{
  "gene_name": "Choline kinase alpha",
  "term_id": "GO:0005737",
  "gene_symbol": "CHKA",
  "gene": "UniProtKB:P35790",
  "term_label": "cytoplasm"
}